siroheme catabolic process [GO:0046157] (biological process) Relationships: is a type of heme catabolic process [GO:0042167] Definition: The chemical reactions and pathways resulting in the breakdown of siroheme, a tetrahydroporphyrin with adjacent, reduced pyrrole rings. Also known as: sirohaem catabolic process, sirohaem catabolism, siroheme breakdown, siroheme catabolism, siroheme degradation Sources: ISBN:0198506732